{
  "term_label": "RISC complex",
  "gene_symbol": "AGO2",
  "gene": "UniProtKB:Q9UKV8",
  "gene_name": "Protein argonaute-2",
  "term_id": "GO:0016442"
}